7-deoxyloganate 7-hydroxylase activity [GO:0140989] (molecular function) Definition: Catalysis of the reaction: 7-deoxyloganate + O2 + reduced [NADPH-hemoprotein reductase] = H+ + H2O + loganate + oxidized [NADPH-hemoprotein reductase]. References: PMID:24710322 Sources: RHEA:57576 Relationships: is a type of oxidoreductase activity, acting on paired donors, with incorporation or reduction of molecular oxygen, reduced flavin or flavoprotein as one donor, and incorporation of one atom of oxygen [GO:0016712]